{
  "term_id": "GO:0004222",
  "gene_name": "A disintegrin and metalloproteinase with thrombospondin motifs 10",
  "gene_symbol": "ADAMTS10",
  "term_label": "metalloendopeptidase activity",
  "gene": "UniProtKB:Q9H324"
}